{
  "term_id": "GO:0005886",
  "gene_name": "Olfactory receptor 2S2",
  "gene_symbol": "OR2S2",
  "gene": "UniProtKB:Q9NQN1",
  "term_label": "plasma membrane"
}